Group III intron splicing [GO:0000374] (biological process) Relationships: is a type of RNA splicing, via transesterification reactions with bulged adenosine as nucleophile [GO:0000377] Definition: The splicing of Group III introns. This occurs by a ribozymic mechanism where the intron sequence forms a distinct 3D structure, characteristic of Group III introns, that is involved in catalyzing the splicing reactions, though protein factors are also required in vivo. Splicing occurs by a series of two transesterification reactions begun by a bulged adenosine residue within the intron sequence as the initiating nucleophile. The intron is excised as a lariat. Though very similar in structure and mechanism to Group II introns, Group III introns are smaller and more streamlined and the splice site consensus sequences are not as well conserved. Note: Note that Group III introns are known to be found in mRNA of plastids of euglenoid protists. Also known as: mRNA splicing References: PMID:11377794 Sources: GOC:krc